regulation of intracellular lipid transport [GO:0032377] (biological process) Sources: GOC:mah Subtypes: negative regulation of intracellular lipid transport [GO:0032378], positive regulation of intracellular lipid transport [GO:0032379], GO:0032380 Definition: Any process that modulates the frequency, rate or extent of the directed movement of lipids within cells. Relationships: is a type of regulation of lipid transport [GO:0032368]; is a type of regulation of intracellular transport [GO:0032386]; regulates intracellular lipid transport [GO:0032365]